{
  "gene": "UniProtKB:P28067",
  "term_id": "GO:0002503",
  "gene_symbol": "HLA-DMA",
  "term_label": "peptide antigen assembly with MHC class II protein complex",
  "gene_name": "HLA class II histocompatibility antigen, DM alpha chain"
}